ephrin receptor signaling pathway [GO:0048013] (biological process) Definition: The series of molecular signals initiated by ephrin binding to its receptor, and ending with the regulation of a downstream cellular process, e.g. transcription. Sources: GOC:ceb Also known as: Eph receptor signaling pathway, Eph receptor signalling pathway Relationships: is a type of cell surface receptor protein tyrosine kinase signaling pathway [GO:0007169] Regulation: regulated by regulation of ephrin receptor signaling pathway [GO:1901187]; negatively regulated by GO:1901188; positively regulated by GO:1901189